{
  "term_label": "positive regulation of toll-like receptor 3 signaling pathway",
  "term_id": "GO:0034141",
  "gene": "UniProtKB:Q8IWB7",
  "gene_symbol": "WDFY1",
  "gene_name": "WD repeat and FYVE domain-containing protein 1"
}